{
  "term_id": "GO:0006265",
  "gene_name": "DNA topoisomerase 3-alpha",
  "gene": "UniProtKB:Q13472",
  "gene_symbol": "TOP3A",
  "term_label": "DNA topological change"
}